response to thyroxine [GO:0097068] (biological process) Relationships: is_a response to amino acid [GO:0043200]; is a type of response to thyroid hormone [GO:0097066]; is_a response to oxygen-containing compound [GO:1901700]; is a type of response to L-phenylalanine derivative [GO:1904386] Also known as: response to T4, response to T4 stimulus, response to thyroxine stimulus Definition: A change in state or activity of a cell or an organism (in terms of movement, secretion, enzyme production, gene expression, etc.) as a result of a thyroxine stimulus. Subtypes: cellular response to thyroxine stimulus [GO:0097069] References: PMID:9916872 Sources: GOC:sjw